{
  "gene_symbol": "ANKRD18B",
  "term_label": "Unknown cellular component",
  "gene": "UniProtKB:A2A2Z9",
  "term_id": "UNKNOWN:0003",
  "gene_name": "Ankyrin repeat domain-containing protein 18B"
}